{
  "gene": "UniProtKB:B6SEH9",
  "term_label": "Unknown cellular component",
  "term_id": "UNKNOWN:0003",
  "gene_symbol": "ERVV-2",
  "gene_name": "Endogenous retrovirus group V member 2 Env polyprotein"
}